{
  "gene": "UniProtKB:Q9C0E4",
  "gene_symbol": "GRIP2",
  "term_label": "Unknown molecular function",
  "term_id": "UNKNOWN:0001",
  "gene_name": "Glutamate receptor-interacting protein 2"
}